{
  "term_id": "GO:0005634",
  "term_label": "nucleus",
  "gene_symbol": "RNF6",
  "gene_name": "E3 ubiquitin-protein ligase RNF6",
  "gene": "UniProtKB:Q9Y252"
}